{
  "gene_name": "BTB_POZ domain-containing protein 9",
  "term_label": "Unknown molecular function",
  "gene_symbol": "BTBD9",
  "term_id": "UNKNOWN:0001",
  "gene": "UniProtKB:Q96Q07"
}